{
  "term_label": "receptor-mediated endocytosis",
  "gene": "UniProtKB:Q86YD5",
  "gene_name": "Low-density lipoprotein receptor class A domain-containing protein 3",
  "gene_symbol": "LDLRAD3",
  "term_id": "GO:0006898"
}